maintenance of organelle location [GO:0051657] (BP) Also known as: maintenance of organelle localization Relationships: is a type of GO:0051651; is part of organelle localization [GO:0051640] Subtypes: maintenance of vesicle location [GO:0051655], GO:0051658, maintenance of mitochondrion location [GO:0051659], GO:0051661, maintenance of Golgi location [GO:0051684], maintenance of ER location [GO:0051685], maintenance of spindle location [GO:0051687], maintenance of plastid location [GO:0051688] Sources: GOC:ai, GOC:dph, GOC:tb Definition: Any process in which an organelle is maintained in a specific location within a cell and prevented from moving elsewhere.